membrane stack [GO:1990007] (cellular component) Definition: A configuration of endoplasmic reticulum (ER) found in Purkinje cells in the cerebellum and in axons in the lateral vestibular nucleus, consisting of parallel and interconnecting tubules whose outer surfaces are covered by particles or ringlike structures. Relationships: is a type of endoplasmic reticulum [GO:0005783] Sources: ISBN:9780195065718, NIF_Subcellular:sao2114874506